{
  "term_label": "Unknown molecular function",
  "gene": "UniProtKB:Q9NZU1",
  "gene_symbol": "FLRT1",
  "term_id": "UNKNOWN:0001",
  "gene_name": "Leucine-rich repeat transmembrane protein FLRT1"
}